{
  "gene": "UniProtKB:Q9Y3A2",
  "gene_symbol": "UTP11",
  "gene_name": "Probable U3 small nucleolar RNA-associated protein 11",
  "term_id": "UNKNOWN:0001",
  "term_label": "Unknown molecular function"
}